chemokine (C-X-C motif) ligand 1 production [GO:0072566] (biological process) Relationships: is_a GO:0032602 Sources: GOC:BHF, GOC:mah Also known as: CXCL1 production, KC production, SCYB1 production, keratinocyte derived chemokine production Regulation: regulated by regulation of chemokine (C-X-C motif) ligand 1 production [GO:2000338]; negatively regulated by negative regulation of chemokine (C-X-C motif) ligand 1 production [GO:2000339]; positively regulated by GO:2000340 Definition: The appearance of chemokine (C-X-C motif) ligand 1 due to biosynthesis or secretion following a cellular stimulus, resulting in an increase in its intracellular or extracellular levels.